{
  "gene_symbol": "SETDB1",
  "gene_name": "Histone-lysine N-methyltransferase SETDB1",
  "gene": "UniProtKB:Q15047",
  "term_label": "heterochromatin organization",
  "term_id": "GO:0070828"
}